{
  "gene": "UniProtKB:Q86TI0",
  "gene_name": "TBC1 domain family member 1",
  "term_id": "GO:0005794",
  "gene_symbol": "TBC1D1",
  "term_label": "Golgi apparatus"
}